{
  "gene": "UniProtKB:Q6UX39",
  "term_id": "GO:0005911",
  "gene_name": "Amelotin",
  "gene_symbol": "AMTN",
  "term_label": "cell-cell junction"
}